{
  "gene": "UniProtKB:Q8NFU0",
  "gene_name": "Bestrophin-4",
  "term_label": "chloride channel activity",
  "gene_symbol": "BEST4",
  "term_id": "GO:0005254"
}